{
  "term_id": "GO:0003899",
  "gene_symbol": "POLR2L",
  "term_label": "DNA-directed RNA polymerase activity",
  "gene": "UniProtKB:P62875",
  "gene_name": "DNA-directed RNA polymerases I, II, and III subunit RPABC5"
}